MAML2-RBP-Jkappa-ICN4 complex [GO:0071178] (cellular component) Also known as: MAML2-RBP-Jkappa-Notch4 complex Relationships: is a type of GO:0140513 Definition: A protein complex that consists of the intracellular domain of Notch4 (ICN4), the DNA-binding transcription factor RBP-Jkappa, and the transcriptional coactivator Mastermind-like-2 (MAML2); the complex is involved in transcriptional activation in response to Notch-mediated signaling. References: PMID:12370315